{
  "term_label": "regulation of alternative mRNA splicing, via spliceosome",
  "term_id": "GO:0000381",
  "gene_name": "Probable RNA-binding protein 19",
  "gene_symbol": "RBM19",
  "gene": "UniProtKB:Q9Y4C8"
}